{
  "term_id": "GO:0005739",
  "gene_symbol": "COX8C",
  "gene_name": "Cytochrome c oxidase subunit 8C, mitochondrial",
  "gene": "UniProtKB:Q7Z4L0",
  "term_label": "mitochondrion"
}